{
  "gene": "UniProtKB:A0A0A0MS02",
  "gene_symbol": "TRGV1",
  "term_label": "Unknown cellular component",
  "term_id": "UNKNOWN:0003",
  "gene_name": "Probable non-functional T cell receptor gamma variable"
}